basidiospore formation [GO:0034295] (biological process) Definition: The process in which spores form outside a specialized end cell known as a basidium. Basidia are characteristic of the basidiomycete fungi (phylum Basidiomycota), and give rise to spores that each contain a haploid nucleus that is the product of meiosis. The spores are usually attached to the basidium by short spikes called sterigmata (singular: sterigma). In most basidiomycetes there are four sterigmata (and four spores) to a basidium. Sources: GOC:di, GOC:ds, GOC:mah, GOC:mcc, https://en.wikipedia.org/wiki/Basidiospore Note: Note that basidiospores and basidia are separate biological structures. The basidium is the structure that bear the basidiospores, but the development of the basidium is a different process than the formation of the basidiospores themselves. For this reason, GO:0034295 basidiospore formation and GO:0075313 basidium development are different terms and are not linked. Relationships: is a type of sexual sporulation resulting in formation of a cellular spore [GO:0043935] Regulation: regulated by regulation of basidiospore formation [GO:0075302]; positively regulated by positive regulation of basidiospore formation [GO:0075303]; negatively regulated by negative regulation of basidiospore formation [GO:0075304]